{
  "term_id": "UNKNOWN:0003",
  "gene_name": "Pecanex-like protein 1",
  "term_label": "Unknown cellular component",
  "gene_symbol": "PCNX1",
  "gene": "UniProtKB:Q96RV3"
}